cell morphogenesis involved in semicircular canal fusion [GO:0060880] (biological process) Sources: GOC:dph, GOC:sdb_2009, GOC:tb Definition: The change in form (cell shape and size) that occurs when a semicircular canal epithelial cell acquires the structural features that allow it to contribute to the process of semicircular canal fusion. Relationships: is a type of cell morphogenesis [GO:0000902]; is a type of embryonic morphogenesis [GO:0048598]; is part of semicircular canal fusion [GO:0060879]